{
  "term_label": "regulation of JNK cascade",
  "gene": "UniProtKB:Q8WTR2",
  "gene_symbol": "DUSP19",
  "term_id": "GO:0046328",
  "gene_name": "Dual specificity protein phosphatase 19"
}